{
  "gene_name": "G-protein coupled receptor 55",
  "term_label": "cannabinoid receptor activity",
  "gene_symbol": "GPR55",
  "term_id": "GO:0004949",
  "gene": "UniProtKB:Q9Y2T6"
}